{
  "term_label": "Unknown molecular function",
  "gene_symbol": "NRSN2",
  "gene": "UniProtKB:Q9GZP1",
  "gene_name": "Neurensin-2",
  "term_id": "UNKNOWN:0001"
}